blood coagulation, fibrin clot formation [GO:0072378] (biological process) References: PMID:26018600 Sources: GOC:add, GOC:mah, GOC:pde Note: See also the biological process term 'blood coagulation, intrinsic pathway ; GO:0007597'. Relationships: is a type of protein activation cascade [GO:0072376]; is part of GO:0007596 Definition: A protein activation cascade that contributes to blood coagulation and consists of the cascade of enzymatic reactions initiated by physical damage to the wall of a blood vessel, leading to the formation of a formation of a fibrin clot at the site of the injury. The process also includes numerous positive and negative regulatory events.